inner mitochondrial membrane organization [GO:0007007] (biological process) Note: See also the cellular component term 'mitochondrial inner membrane ; GO:0005743'. Relationships: is a type of GO:0007006 Also known as: inner mitochondrial membrane organisation, mitochondrial inner membrane organization, inner mitochondrial membrane organization and biogenesis Definition: A process that is carried out at the cellular level which results in the assembly, arrangement of constituent parts, or disassembly of the mitochondrial inner membrane. Subtypes: cristae formation [GO:0042407], protein insertion into mitochondrial inner membrane [GO:0045039], mitochondrial inner membrane fusion [GO:1990627] Sources: GOC:ai, GOC:dph, GOC:jl, GOC:mah